{
  "gene": "UniProtKB:Q9BV81",
  "gene_symbol": "EMC6",
  "gene_name": "ER membrane protein complex subunit 6",
  "term_id": "GO:0000045",
  "term_label": "autophagosome assembly"
}